{
  "gene_name": "Lethal(3)malignant brain tumor-like protein 4",
  "term_label": "histone binding",
  "term_id": "GO:0042393",
  "gene_symbol": "L3MBTL4",
  "gene": "UniProtKB:Q8NA19"
}